{
  "gene_symbol": "EDN2",
  "gene_name": "Endothelin-2",
  "term_id": "GO:0045987",
  "gene": "UniProtKB:P20800",
  "term_label": "positive regulation of smooth muscle contraction"
}